{
  "term_label": "glutathione peroxidase activity",
  "gene": "UniProtKB:P36969",
  "gene_name": "Phospholipid hydroperoxide glutathione peroxidase",
  "gene_symbol": "GPX4",
  "term_id": "GO:0004602"
}